{
  "term_label": "olfactory receptor activity",
  "term_id": "GO:0004984",
  "gene_name": "Olfactory receptor 4D10",
  "gene": "UniProtKB:Q8NGI6",
  "gene_symbol": "OR4D10"
}